taurine-2-oxoglutarate transaminase activity [GO:0050322] (molecular function) Relationships: is a type of GO:0008483 References: PMID:16535664 Sources: RHEA:16353 Definition: Catalysis of the reaction: taurine + 2-oxoglutarate = sulfoacetaldehyde + L-glutamate. Also known as: taurine aminotransferase activity, taurine transaminase activity, taurine--alpha-ketoglutarate aminotransferase activity, taurine--glutamate transaminase activity, taurine:2-oxoglutarate aminotransferase activity